{
  "gene_name": "Disintegrin and metalloproteinase domain-containing protein 32",
  "term_label": "metalloendopeptidase activity",
  "term_id": "GO:0004222",
  "gene_symbol": "ADAM32",
  "gene": "UniProtKB:Q8TC27"
}